negative regulation of Toll signaling pathway [GO:0045751] (biological process) Sources: GOC:go_curators Relationships: is a type of regulation of Toll signaling pathway [GO:0008592]; is a type of negative regulation of signal transduction [GO:0009968]; RO_0002212 GO:0008063 Definition: Any process that stops, prevents, or reduces the frequency, rate or extent of the Tl signaling pathway. Also known as: down regulation of Toll signaling pathway, down-regulation of Toll signaling pathway, downregulation of Toll signaling pathway, negative regulation of Tl signaling pathway, negative regulation of Tl signalling pathway, inhibition of Toll signaling pathway